RNA polymerase I promoter clearance [GO:0001182] (biological process) Also known as: RNA polymerase I promoter escape, promoter clearance from RNA polymerase I promoter, promoter clearance from RNA polymerase I promoter for nuclear large rRNA transcript References: PMID:18559419 Sources: GOC:txnOH Relationships: is a type of promoter clearance during DNA-templated transcription [GO:0001109]; is part of transcription by RNA polymerase I [GO:0006360] Definition: A process that mediates the transition from the initiation to the elongation phases of transcription by RNA polymerase I, generally including a conformational change from the initiation conformation to the elongation conformation. Promoter clearance often involves breaking contact with transcription factors involved only in the initiation phase and making contacts with elongation specific factors.